{
  "gene_name": "Ubiquilin-1",
  "gene_symbol": "UBQLN1",
  "term_id": "GO:0031593",
  "term_label": "polyubiquitin modification-dependent protein binding",
  "gene": "UniProtKB:Q9UMX0"
}